{
  "term_id": "UNKNOWN:0001",
  "gene_name": "Protein FAM131A",
  "gene": "UniProtKB:Q6UXB0",
  "term_label": "Unknown molecular function",
  "gene_symbol": "FAM131A"
}